{
  "gene": "UniProtKB:P55795",
  "gene_name": "Heterogeneous nuclear ribonucleoprotein H2",
  "gene_symbol": "HNRNPH2",
  "term_label": "RNA binding",
  "term_id": "GO:0003723"
}